{
  "term_id": "GO:0016015",
  "gene": "UniProtKB:O95813",
  "gene_name": "Cerberus",
  "term_label": "morphogen activity",
  "gene_symbol": "CER1"
}